{
  "gene_symbol": "GAPDHS",
  "gene": "UniProtKB:O14556",
  "term_id": "GO:0005829",
  "term_label": "cytosol",
  "gene_name": "Glyceraldehyde-3-phosphate dehydrogenase, testis-specific"
}